{
  "gene": "UniProtKB:P39210",
  "term_label": "cytoplasm",
  "term_id": "GO:0005737",
  "gene_name": "Protein Mpv17",
  "gene_symbol": "MPV17"
}